{
  "gene_name": "Heme oxygenase 1",
  "term_label": "endoplasmic reticulum",
  "gene": "UniProtKB:P09601",
  "term_id": "GO:0005783",
  "gene_symbol": "HMOX1"
}